{
  "term_id": "GO:0031647",
  "gene_name": "Ubiquitin carboxyl-terminal hydrolase 13",
  "gene_symbol": "USP13",
  "term_label": "regulation of protein stability",
  "gene": "UniProtKB:Q92995"
}